pyranose dehydrogenase (acceptor) activity [GO:0033718] (molecular function) Also known as: PDH, pyranose dehydrogenase activity, pyranose-quinone oxidoreductase activity, pyranose:acceptor oxidoreductase activity, quinone-dependent pyranose dehydrogenase activity Definition: Catalysis of the reactions: pyranose + acceptor = 2-dehydropyranose (or 3-dehydropyranose or 2,3-didehydropyranose) + reduced acceptor, and a pyranoside + acceptor = a 3-dehydropyranoside (or 3,4-didehydropyranoside) + reduced acceptor. Sources: EC:1.1.99.29 Relationships: is a type of oxidoreductase activity, acting on CH-OH group of donors [GO:0016614]